{
  "term_label": "Unknown biological process",
  "term_id": "UNKNOWN:0002",
  "gene": "UniProtKB:P53370",
  "gene_symbol": "NUDT6",
  "gene_name": "Nucleoside diphosphate-linked moiety X motif 6"
}